positive regulation of macrophage derived foam cell differentiation [GO:0010744] (biological process) Sources: GOC:add, GOC:dph, GOC:tb Definition: Any process that increases the rate, frequency or extent of macrophage derived foam cell differentiation. Macrophage derived foam cell differentiation is the process in which a macrophage acquires the specialized features of a foam cell. A foam cell is a type of cell containing lipids in small vacuoles and typically seen in atherosclerotic lesions, as well as other conditions. Relationships: is a type of regulation of macrophage derived foam cell differentiation [GO:0010743]; is_a GO:0045597; positively regulates macrophage derived foam cell differentiation [GO:0010742]